{
  "gene_symbol": "BATF3",
  "term_label": "regulation of transcription by RNA polymerase II",
  "term_id": "GO:0006357",
  "gene_name": "Basic leucine zipper transcriptional factor ATF-like 3",
  "gene": "UniProtKB:Q9NR55"
}